L-lysine transmembrane transporter activity [GO:0015189] (molecular function) Definition: Enables the transfer of L-lysine from one side of a membrane to the other. L-lysine is 2,6-diaminohexanoic acid. Sources: GOC:ai, GOC:mtg_transport, ISBN:0815340729 Also known as: histidine/arginine/lysine/ornithine porter activity, L-lysine permease, lysine permease activity Relationships: is a type of GO:0015174; is a type of GO:0015179; is part of L-lysine transmembrane transport [GO:1903401] Subtypes: high-affinity lysine transmembrane transporter activity [GO:0005292], GO:0015661, GO:0106439